heart contraction [GO:0060047] (biological process) Definition: The multicellular organismal process in which the heart decreases in volume in a characteristic way to propel blood through the body. Sources: GOC:dph Also known as: heart beating, cardiac contraction, hemolymph circulation Relationships: is_a GO:0003015; is part of blood circulation [GO:0008015] Regulation: regulated by regulation of heart contraction [GO:0008016]; negatively regulated by negative regulation of heart contraction [GO:0045822]; positively regulated by positive regulation of heart contraction [GO:0045823]